{
  "gene_symbol": "TRAV9-2",
  "term_id": "UNKNOWN:0001",
  "term_label": "Unknown molecular function",
  "gene": "UniProtKB:A0A087WT02",
  "gene_name": "T cell receptor alpha variable 9-2"
}